{
  "gene_symbol": "VCX",
  "term_id": "GO:0007420",
  "gene": "UniProtKB:Q9H320",
  "term_label": "brain development",
  "gene_name": "Variable charge X-linked protein 1"
}